{
  "gene_name": "Molybdenum cofactor sulfurase",
  "gene": "UniProtKB:Q96EN8",
  "term_id": "GO:0008265",
  "gene_symbol": "MOCOS",
  "term_label": "molybdenum cofactor sulfurtransferase activity"
}